specification of metanephric distal tubule identity [GO:0072295] (biological process) Definition: The process in which the distal tubule of the metanephric nephron acquires its identity. Sources: GOC:bf, GOC:mtg_kidney_jan10 Relationships: is a type of specification of distal tubule identity [GO:0072084]; is a type of GO:0072293; is part of GO:0072287